{
  "gene": "UniProtKB:O75781",
  "gene_symbol": "PALM",
  "gene_name": "Paralemmin-1",
  "term_label": "adenylate cyclase-inhibiting G protein-coupled receptor signaling pathway",
  "term_id": "GO:0007193"
}